{
  "gene_name": "Nuclear receptor subfamily 0 group B member 1",
  "gene": "UniProtKB:P51843",
  "gene_symbol": "NR0B1",
  "term_id": "GO:0005634",
  "term_label": "nucleus"
}